{
  "term_id": "GO:0016176",
  "gene_symbol": "NCF2",
  "term_label": "superoxide-generating NADPH oxidase activator activity",
  "gene": "UniProtKB:P19878",
  "gene_name": "Neutrophil cytosol factor 2"
}